{
  "gene": "UniProtKB:P13805",
  "term_label": "troponin T binding",
  "term_id": "GO:0031014",
  "gene_name": "Troponin T, slow skeletal muscle",
  "gene_symbol": "TNNT1"
}